positive regulation of secretion of lysosomal enzymes [GO:0090340] (biological process) Sources: GOC:BHF Definition: Any process that increases the rate, frequency or extent of secretion of lysosomal enzymes, the controlled release of lysosomal enzymes by a cell. Relationships: is a type of positive regulation of protein secretion [GO:0050714]; is a type of regulation of secretion of lysosomal enzymes [GO:0090182]; positively regulates secretion of lysosomal enzymes [GO:0033299]